{
  "gene_name": "EVI5-like protein",
  "term_id": "GO:0005096",
  "term_label": "GTPase activator activity",
  "gene": "UniProtKB:Q96CN4",
  "gene_symbol": "EVI5L"
}